{
  "term_id": "GO:0000932",
  "term_label": "P-body",
  "gene_symbol": "DCP1A",
  "gene": "UniProtKB:Q9NPI6",
  "gene_name": "mRNA-decapping enzyme 1A"
}